{
  "term_label": "microtubule-based movement",
  "gene_name": "Kinesin-like protein KIF20A",
  "gene_symbol": "KIF20A",
  "gene": "UniProtKB:O95235",
  "term_id": "GO:0007018"
}